dinoflagellate antapical horn [GO:0097687] (CC) Definition: A horn-shaped dinoflagellate antapex found in thecate species. References: PMID:7002229 Sources: GOC:at Relationships: is a type of dinoflagellate antapex [GO:0097684]